COPII-coated vesicle lumen [GO:0106173] (cellular component) Definition: The volume enclosed by the membrane of a COPII-coated endocytic vesicle. Relationships: is a type of cytoplasmic vesicle lumen [GO:0060205] References: PMID:21172817 Sources: GOC:pde